{
  "gene_name": "Sodium-independent sulfate anion transporter",
  "gene_symbol": "SLC26A11",
  "term_id": "GO:0005886",
  "gene": "UniProtKB:Q86WA9",
  "term_label": "plasma membrane"
}